delta DNA polymerase complex [GO:0043625] (cellular component) Definition: A multimeric DNA polymerase enzyme complex which differs in composition amongst species; in humans it is a heterotetramer of four subunits of approximately 125, 50, 68 and 12kDa, while in S. cerevisiae, it has three different subunits which form a heterotrimer, and the active enzyme is a dimer of this heterotrimer. Functions in DNA replication, mismatch repair and excision repair. References: PMID:11205330, PMID:12403614 Sources: GOC:jl, ISBN:0198547684 Also known as: delta-DNA polymerase complex Relationships: is a type of DNA polymerase complex [GO:0042575]; is a type of nuclear protein-containing complex [GO:0140513]; is part of nuclear replisome [GO:0043601]